betaine-aldehyde dehydrogenase (NAD+) activity [GO:0008802] (molecular function) Also known as: BADH activity, BetB, betaine aldehyde dehydrogenase activity, betaine aldehyde oxidase activity, betaine-aldehyde:NAD+ oxidoreductase activity Relationships: is a type of aldehyde dehydrogenase (NAD+) activity [GO:0004029] Sources: EC:1.2.1.8 Definition: Catalysis of the reaction: betaine aldehyde + NAD+ + H2O = betaine + NADH + H+.